regulation of isoprene biosynthetic process [GO:1900947] (biological process) Relationships: is a type of regulation of isoprenoid metabolic process [GO:0019747]; is a type of regulation of lipid biosynthetic process [GO:0046890]; is a type of GO:1900911; regulates isoprene biosynthetic process [GO:0043612] Also known as: regulation of 2-methyl-1,3-butadiene biosynthesis, regulation of 2-methyl-1,3-butadiene biosynthetic process, regulation of hemiterpene biosynthesis, regulation of hemiterpene biosynthetic process Sources: GOC:TermGenie, GOC:mengo_curators Definition: Any process that modulates the frequency, rate or extent of isoprene biosynthetic process. Subtypes: negative regulation of isoprene biosynthetic process [GO:1900948], positive regulation of isoprene biosynthetic process [GO:1900949]